{
  "term_id": "GO:0030121",
  "term_label": "AP-1 adaptor complex",
  "gene_symbol": "STON2",
  "gene_name": "Stonin-2",
  "gene": "UniProtKB:Q8WXE9"
}